{
  "gene_symbol": "SRCIN1",
  "gene": "UniProtKB:Q9C0H9",
  "term_label": "cytoplasm",
  "term_id": "GO:0005737",
  "gene_name": "SRC kinase signaling inhibitor 1"
}